{
  "term_label": "immunoglobulin mediated immune response",
  "gene_symbol": "IGHV4-38-2",
  "gene": "UniProtKB:P0DP08",
  "term_id": "GO:0016064",
  "gene_name": "Immunoglobulin heavy variable 4-38-2"
}